calcidiol 1-monooxygenase activity [GO:0004498] (molecular function) Definition: Catalysis of the reaction: calcidiol + H+ + NADPH + O2 = calcitriol + H2O + NADP+. Sources: EC:1.14.15.18, RHEA:20573 Relationships: is a type of oxidoreductase activity, acting on paired donors, with incorporation or reduction of molecular oxygen, NAD(P)H as one donor, and incorporation of one atom of oxygen [GO:0016709]; BFO_0000050 calcitriol biosynthetic process from calciol [GO:0036378] Also known as: 25-hydroxy vitamin D3 1-alpha-hydroxylase activity, 25-hydroxycholecalciferol 1-hydroxylase activity, calcidiol,NADPH:oxygen oxidoreductase (1-hydroxylating), cytochrome P450 CYP27B, 1-hydroxylase-25-hydroxyvitamin D3 activity, 25-OHD-1 alpha-hydroxylase activity, 25-hydroxy D3-1alpha-hydroxylase activity, 25-hydroxycholecalciferol 1-monooxygenase activity, 25-hydroxycholecalciferol 1alpha-hydroxylase activity, 25-hydroxycholecalciferol-1-hydroxylase activity, 25-hydroxyvitamin D-1 alpha hydroxylase activity, 25-hydroxyvitamin D3 1alpha-hydroxylase activity